{
  "term_label": "Unknown biological process",
  "gene_symbol": "PVALB",
  "gene_name": "Parvalbumin alpha",
  "gene": "UniProtKB:P20472",
  "term_id": "UNKNOWN:0002"
}